{
  "term_id": "UNKNOWN:0002",
  "gene_symbol": "ARL2BP",
  "gene_name": "ADP-ribosylation factor-like protein 2-binding protein",
  "term_label": "Unknown biological process",
  "gene": "UniProtKB:Q9Y2Y0"
}